tRNA 2-selenouridine synthase activity [GO:0043828] (molecular function) Definition: Catalysis of the reaction: 5-methylaminomethyl-2-thiouridine + selenophosphate = 5-methylaminomethyl-2-selenouridine + phosphate (at the wobble position in tRNA). References: PMID:14594807 Sources: RHEA:42716 Relationships: is a type of selenotransferase activity [GO:0016785]; is a type of catalytic activity, acting on a tRNA [GO:0140101]